oxidoreductase activity, acting on paired donors, with oxidation of a pair of donors resulting in the reduction of molecular oxygen to two molecules of water [GO:0016717] (molecular function) Subtypes: acyl-CoA desaturase activity [GO:0016215], acyl-lipid Delta(12)-acetylenase [GO:0016720], sphingolipid delta-4 desaturase activity [GO:0042284], stearoyl-[ACP] desaturase activity [GO:0045300], (S)-stylopine synthase activity [GO:0047052], (S)-cheilanthifoline synthase activity [GO:0047053], GO:0047054, salutaridine synthase activity [GO:0047055], (S)-canadine synthase activity [GO:0047056], acyl-lipid omega-6 desaturase (cytochrome b5) activity [GO:0050184], GO:0050207, GO:0052631, sterol desaturase activity [GO:0070704], GO:0102003, GO:0102431, (S)-nandinine synthase activity [GO:0102632], palmitoyl-[glycerolipid] 3-(E)-desaturase activity [GO:0102654], GO:0102843, acyl-lipid (n+3)-(Z)-desaturase (ferredoxin) activity [GO:0102850], acyl-lipid omega-3 desaturase (cytochrome b5) activity [GO:0102859], delta6-acyl-lipid desaturase activity [GO:0102865], acyl-lipid (8-3)-desaturase activity [GO:0102866], (S)-corytuberine synthase activity [GO:0102963], sn-2 acyl-lipid omega-3 desaturase (ferredoxin) activity [GO:0102993], versicolorin B desaturase activity [GO:0140398] Relationships: is a type of GO:0016705 Definition: Catalysis of an oxidation-reduction (redox) reaction in which hydrogen or electrons are transferred from each of two donors, and molecular oxygen is reduced to two molecules of water. Sources: EC:1.14.19.-